{
  "gene_symbol": "BAP1",
  "gene": "UniProtKB:Q92560",
  "term_id": "GO:0005737",
  "gene_name": "Ubiquitin carboxyl-terminal hydrolase BAP1",
  "term_label": "cytoplasm"
}